{
  "gene": "UniProtKB:P17025",
  "gene_name": "Zinc finger protein 182",
  "gene_symbol": "ZNF182",
  "term_label": "DNA-binding transcription factor activity, RNA polymerase II-specific",
  "term_id": "GO:0000981"
}